{
  "term_id": "GO:0009986",
  "term_label": "cell surface",
  "gene_name": "Integrin alpha-9",
  "gene": "UniProtKB:Q13797",
  "gene_symbol": "ITGA9"
}